{
  "gene_symbol": "HDAC4",
  "gene": "UniProtKB:P56524",
  "term_label": "histone deacetylase activity",
  "term_id": "GO:0004407",
  "gene_name": "Histone deacetylase 4"
}